{
  "gene": "UniProtKB:P56705",
  "gene_symbol": "WNT4",
  "term_id": "GO:0005125",
  "gene_name": "Protein Wnt-4",
  "term_label": "cytokine activity"
}